{
  "gene": "UniProtKB:Q96KM6",
  "term_id": "UNKNOWN:0002",
  "gene_name": "Zinc finger protein 512B",
  "term_label": "Unknown biological process",
  "gene_symbol": "ZNF512B"
}